{
  "term_id": "GO:0000981",
  "gene_name": "Zinc finger protein 675",
  "term_label": "DNA-binding transcription factor activity, RNA polymerase II-specific",
  "gene": "UniProtKB:Q8TD23",
  "gene_symbol": "ZNF675"
}